DNA strand displacement [GO:0000732] (biological process) Relationships: is a type of DNA metabolic process [GO:0006259]; is part of DNA recombination [GO:0006310] References: PMID:10357855 Also known as: strand displacement, D-loop dissociation, D-loop processing, displacement loop dissociation, displacement loop processing Definition: The rejection of the broken 3' single-strand DNA molecule that formed heteroduplex DNA with its complement in an intact duplex DNA. The Watson-Crick base pairing in the original duplex is restored. The rejected 3' single-strand DNA molecule reanneals with its original complement to reform two intact duplex molecules. Subtypes: GO:0000714